paraxial mesodermal cell fate specification [GO:0048348] (biological process) Regulation: regulated by regulation of paraxial mesodermal cell fate specification [GO:0048349]; RO_0002213 by GO:0048350; RO_0002212 by negative regulation of paraxial mesodermal cell fate specification [GO:0048351] Definition: The process in which a cell becomes capable of differentiating autonomously into a paraxial mesoderm cell in an environment that is neutral with respect to the developmental pathway; upon specification, the cell fate can be reversed. Sources: GOC:dgh Relationships: is a type of mesodermal cell fate specification [GO:0007501]; BFO_0000050 GO:0048343